{
  "gene": "UniProtKB:Q10567",
  "term_label": "Unknown cellular component",
  "gene_name": "AP-1 complex subunit beta-1",
  "term_id": "UNKNOWN:0003",
  "gene_symbol": "AP1B1"
}